{
  "gene": "UniProtKB:P56706",
  "term_id": "GO:0005125",
  "gene_name": "Protein Wnt-7b",
  "gene_symbol": "WNT7B",
  "term_label": "cytokine activity"
}